NLRP3 inflammasome complex assembly [GO:0044546] (BP) Regulation: RO_0002211 by GO:1900225; negatively regulated by negative regulation of NLRP3 inflammasome complex assembly [GO:1900226]; RO_0002213 by positive regulation of NLRP3 inflammasome complex assembly [GO:1900227] References: PMID:21048113 Sources: GOC:jl Relationships: is a type of canonical inflammasome complex assembly [GO:0140632] Definition: The aggregation, arrangement and bonding together of a set of components to form the NLRP3 inflammasome complex, occurring at the level of an individual cell. Also known as: NALP3 inflammasome complex assembly, NLRP3 inflammasome activation